{
  "term_id": "UNKNOWN:0002",
  "gene_name": "Centrosomal protein of 104 kDa",
  "gene": "UniProtKB:O60308",
  "term_label": "Unknown biological process",
  "gene_symbol": "CEP104"
}